microtubule polymerization based protein transport to cell tip cortex [GO:0099110] (biological process) Relationships: is a type of microtubule polymerization based protein transport [GO:0099112]; is a type of protein localization to cell cortex of cell tip [GO:1990896] References: PMID:11018050 Sources: GOC:dos, GOC:vw Definition: The transport of a protein to the cortex of the cell tip, driven by polymerization of a microtubule to which the protein is attached.